protein lipidation [GO:0006497] (biological process) Sources: GOC:jl Note: For non-covalent interactions with a lipid, consider instead the term 'lipid binding ; GO:0008289' and its children. Regulation: RO_0002211 by GO:1903059; negatively regulated by negative regulation of protein lipidation [GO:1903060]; positively regulated by positive regulation of protein lipidation [GO:1903061] Definition: The covalent attachment of lipid groups to an amino acid in a protein. Also known as: lipid:protein modification, protein amino acid lipidation Relationships: is a type of protein modification process [GO:0036211]; is part of GO:0042158 Subtypes: N-terminal protein lipidation [GO:0006498], C-terminal protein lipidation [GO:0006501], protein octanoylation [GO:0018190], protein palmitoylation [GO:0018345], GO:0018377, protein palmitoleylation [GO:0045234], protein decanoylation [GO:0051366], protein stearoylation [GO:0140438]